fatty acid beta-oxidation multienzyme complex [GO:0036125] (cellular component) Definition: A multienzyme complex possessing three kinds of enzymes that catalyze the chain reactions in the fatty acid beta-oxidation cycle, enoyl-CoA hydratase (ECH), 3-hydroxyacyl-CoA dehydrogenase (HACD), and acetyl-CoA C-acyltransferase (KACT). Relationships: is a type of oxidoreductase complex [GO:1990204]; is a type of transferase complex [GO:1990234] Subtypes: GO:0016507 References: PMID:12115060, PMID:16472743 Sources: GOC:imk Note: For fatty acid beta-oxidation multienzyme complexes located in the mitochondrial matrix, consider instead the term 'mitochondrial fatty acid beta-oxidation multienzyme complex ; GO:0016507'.